{
  "term_id": "GO:0000978",
  "gene": "UniProtKB:Q12837",
  "term_label": "RNA polymerase II cis-regulatory region sequence-specific DNA binding",
  "gene_name": "POU domain, class 4, transcription factor 2",
  "gene_symbol": "POU4F2"
}